{
  "gene": "UniProtKB:O75310",
  "gene_symbol": "UGT2B11",
  "term_label": "Unknown cellular component",
  "term_id": "UNKNOWN:0003",
  "gene_name": "UDP-glucuronosyltransferase 2B11"
}